{
  "term_label": "microtubule-based movement",
  "gene_symbol": "DYNLRB1",
  "term_id": "GO:0007018",
  "gene_name": "Dynein light chain roadblock-type 1",
  "gene": "UniProtKB:Q9NP97"
}